{
  "term_label": "mitochondrial electron transport, succinate to ubiquinone",
  "gene_symbol": "SDHAF2",
  "gene_name": "Succinate dehydrogenase assembly factor 2, mitochondrial",
  "gene": "UniProtKB:Q9NX18",
  "term_id": "GO:0006121"
}